{
  "gene_name": "Calcyclin-binding protein",
  "gene": "UniProtKB:Q9HB71",
  "term_label": "SCF ubiquitin ligase complex",
  "term_id": "GO:0019005",
  "gene_symbol": "CACYBP"
}